{
  "gene_symbol": "ENTHD1",
  "gene": "UniProtKB:Q8IYW4",
  "term_label": "endocytosis",
  "term_id": "GO:0006897",
  "gene_name": "ENTH domain-containing protein 1"
}